{
  "gene_name": "Metal transporter CNNM3",
  "term_id": "GO:0022857",
  "gene_symbol": "CNNM3",
  "term_label": "transmembrane transporter activity",
  "gene": "UniProtKB:Q8NE01"
}